P6 peroxisome [GO:0019824] (cellular component) Also known as: peroxisome vesicle Relationships: is_a peroxisome [GO:0005777] Note: Note that this peroxisome assembly pathway is described in the yeast Yarrowia lipolytica. See also the cellular component terms 'P1 peroxisome ; GO:0019819', 'P2 peroxisome ; GO:0019820', 'P3 peroxisome ; GO:0019821', 'P4 peroxisome ; GO:0019822', and 'P5 peroxisome ; GO:0019823'. Definition: A subform of peroxisome that corresponds to an intermediate in a peroxisome assembly pathway, which operates by conversion of peroxisomal subforms in the direction P1, P2 -> P3 -> P4 -> P5 -> P6. P6 peroxisomes are distinguished from the other subforms on the bases of buoyant density and protein content, and are equivalent to mature peroxisomes. References: PMID:10629216